negative regulation of calcium-mediated signaling [GO:0050849] (biological process) Subtypes: negative regulation of calcineurin-mediated signaling [GO:0106057], negative regulation of CAMKK-AMPK signaling cascade [GO:1905290] Relationships: is a type of regulation of calcium-mediated signaling [GO:0050848]; is a type of negative regulation of intracellular signal transduction [GO:1902532]; negatively regulates calcium-mediated signaling [GO:0019722] Definition: Any process that stops, prevents, or reduces the frequency, rate or extent of calcium-mediated signaling. References: PMID:11696592 Sources: GOC:ai Also known as: down regulation of calcium-mediated signaling, down-regulation of calcium-mediated signaling, downregulation of calcium-mediated signaling, negative regulation of calcium-mediated signalling, inhibition of calcium-mediated signaling